{
  "gene_name": "Neuropeptide Y receptor type 1",
  "gene": "UniProtKB:P25929",
  "term_label": "neuron projection",
  "term_id": "GO:0043005",
  "gene_symbol": "NPY1R"
}